{
  "gene_symbol": "WFDC9",
  "term_label": "innate immune response",
  "gene_name": "Protein WFDC9",
  "gene": "UniProtKB:Q8NEX5",
  "term_id": "GO:0045087"
}